{
  "term_label": "regulation of non-canonical NF-kappaB signal transduction",
  "gene_symbol": "BCL3",
  "term_id": "GO:1901222",
  "gene": "UniProtKB:P20749",
  "gene_name": "B-cell lymphoma 3 protein"
}